lipid phosphorylation [GO:0046834] (biological process) Sources: GOC:bf, ISBN:0198506732 Definition: The process of introducing one or more phosphate groups into a lipid, any member of a group of substances soluble in lipid solvents but only sparingly soluble in aqueous solvents. Relationships: is_a GO:0016310; is a type of lipid modification [GO:0030258]